{
  "term_label": "microfilament motor activity",
  "term_id": "GO:0000146",
  "gene_name": "Myosin-9",
  "gene": "UniProtKB:P35579",
  "gene_symbol": "MYH9"
}